{
  "gene": "UniProtKB:Q9NVL8",
  "term_label": "Unknown molecular function",
  "term_id": "UNKNOWN:0001",
  "gene_name": "Uncharacterized protein CCDC198",
  "gene_symbol": "CCDC198"
}